{
  "gene_symbol": "CYSRT1",
  "gene": "UniProtKB:A8MQ03",
  "term_id": "UNKNOWN:0001",
  "term_label": "Unknown molecular function",
  "gene_name": "Cysteine-rich tail protein 1"
}